{
  "gene_symbol": "CRLF1",
  "gene_name": "Cytokine receptor-like factor 1",
  "gene": "UniProtKB:O75462",
  "term_id": "GO:0019221",
  "term_label": "cytokine-mediated signaling pathway"
}